{
  "gene": "UniProtKB:P45985",
  "term_label": "MAPK cascade",
  "term_id": "GO:0000165",
  "gene_symbol": "MAP2K4",
  "gene_name": "Dual specificity mitogen-activated protein kinase kinase 4"
}